negative regulation of F-9775B biosynthetic process [GO:1900676] (biological process) Definition: Any process that stops, prevents or reduces the frequency, rate or extent of F-9775B biosynthetic process. Also known as: down regulation of F-9775B anabolism, down regulation of F-9775B biosynthesis, down regulation of F-9775B biosynthetic process, down regulation of F-9775B formation, down regulation of F-9775B synthesis, down-regulation of F-9775B anabolism, down-regulation of F-9775B biosynthesis, down-regulation of F-9775B biosynthetic process, down-regulation of F-9775B formation, down-regulation of F-9775B synthesis, downregulation of F-9775B anabolism, downregulation of F-9775B biosynthesis, downregulation of F-9775B biosynthetic process, downregulation of F-9775B formation, downregulation of F-9775B synthesis, inhibition of F-9775B anabolism, inhibition of F-9775B biosynthesis, inhibition of F-9775B formation, inhibition of F-9775B synthesis, negative regulation of F-9775B anabolism, negative regulation of F-9775B biosynthesis, negative regulation of F-9775B formation, negative regulation of F-9775B synthesis, inhibition of F-9775B biosynthetic process Sources: GOC:TermGenie, GOC:di Relationships: is a type of GO:1900675; is a type of negative regulation of polyketide biosynthetic process [GO:1900733]; negatively regulates F-9775B biosynthetic process [GO:1900614]